{
  "term_id": "GO:0005634",
  "gene_symbol": "NSUN2",
  "gene": "UniProtKB:Q08J23",
  "term_label": "nucleus",
  "gene_name": "RNA cytosine C(5)-methyltransferase NSUN2"
}